methylseleninic acid reductase activity [GO:0098626] (molecular function) Definition: Catalysis of the reaction: NADPH + H+ + CH3SeO2H = NADP+ + CH3SeOH + H2O. References: PMID:11782468 Relationships: is a type of oxidoreductase activity, acting on NAD(P)H [GO:0016651]